{
  "term_label": "nuclear origin of replication recognition complex",
  "gene_name": "Origin recognition complex subunit 3",
  "gene_symbol": "ORC3",
  "gene": "UniProtKB:Q9UBD5",
  "term_id": "GO:0005664"
}